regulation of mitotic sister chromatid segregation [GO:0033047] (biological process) Relationships: is a type of GO:0033045; regulates GO:0000070 Definition: Any process that modulates the frequency, rate or extent of sister chromatid segregation during mitosis. Sources: GOC:mah Subtypes: negative regulation of mitotic sister chromatid segregation [GO:0033048], GO:0062033, regulation of mitotic cell cycle spindle assembly checkpoint [GO:0090266], regulation of attachment of mitotic spindle microtubules to kinetochore [GO:1902423]